{
  "gene_name": "Trimeric intracellular cation channel type A",
  "term_label": "potassium channel activity",
  "gene": "UniProtKB:Q9H6F2",
  "gene_symbol": "TMEM38A",
  "term_id": "GO:0005267"
}